allantoin catabolic process [GO:0000256] (biological process) Sources: GOC:mah, ISBN:0198547684 Definition: The chemical reactions and pathways resulting in the breakdown of allantoin, (2,5-dioxo-4-imidazolidinyl)urea. Relationships: is a type of allantoin metabolic process [GO:0000255]; is a type of amide catabolic process [GO:0043605] Subtypes: allantoin assimilation pathway [GO:0009442] Also known as: allantoin breakdown, allantoin catabolism, allantoin degradation